peptidyl-serine octanoylation [GO:0018191] (biological process) Relationships: is a type of protein octanoylation [GO:0018190]; is a type of peptidyl-serine modification [GO:0018209] Definition: The octanoylation of peptidyl-serine to form peptidyl-O3-octanoyl-L-serine, typical of the protein ghrelin. References: PMID:10604470 Sources: RESID:AA0290